{
  "gene_symbol": "STARD10",
  "term_id": "UNKNOWN:0002",
  "term_label": "Unknown biological process",
  "gene": "UniProtKB:Q9Y365",
  "gene_name": "START domain-containing protein 10"
}